{
  "term_label": "extracellular space",
  "gene_symbol": "CRISPLD2",
  "gene": "UniProtKB:Q9H0B8",
  "term_id": "GO:0005615",
  "gene_name": "Cysteine-rich secretory protein LCCL domain-containing 2"
}